{
  "gene_symbol": "WNK3",
  "term_label": "cytosol",
  "gene_name": "Serine_threonine-protein kinase WNK3",
  "term_id": "GO:0005829",
  "gene": "UniProtKB:Q9BYP7"
}